host cell cytosol [GO:0044164] (cellular component) Relationships: is_a GO:0033655 Also known as: host cytosol Definition: The part of the host cell cytoplasm that does not contain organelles but which does contain other particulate matter, such as protein complexes. Sources: GOC:jl